rhombomere 6 structural organization [GO:0021668] (biological process) Definition: The process that contributes to creating the structural organization of rhombomere 6. This process pertains to the physical shaping of a rudimentary structure. Rhombomeres are transverse segments of the developing rhombencephalon. Rhombomeres are lineage restricted, express different genes from one another, and adopt different developmental fates. Rhombomeres are numbered in an anterior to posterior order. Sources: GOC:cls, GOC:dgh, GOC:dph, GOC:jid, GO_REF:0000021 Relationships: is_a GO:0021595; is part of rhombomere 6 morphogenesis [GO:0021667] Also known as: rhombomere 6 structural organisation